{
  "gene": "UniProtKB:Q92922",
  "term_label": "positive regulation of DNA-templated transcription",
  "gene_symbol": "SMARCC1",
  "term_id": "GO:0045893",
  "gene_name": "SWI_SNF complex subunit SMARCC1"
}